{
  "gene": "UniProtKB:P98171",
  "term_id": "GO:0005096",
  "term_label": "GTPase activator activity",
  "gene_symbol": "ARHGAP4",
  "gene_name": "Rho GTPase-activating protein 4"
}